{
  "gene": "UniProtKB:Q9Y508",
  "gene_symbol": "RNF114",
  "term_id": "GO:0000209",
  "gene_name": "E3 ubiquitin-protein ligase RNF114",
  "term_label": "protein polyubiquitination"
}